{
  "gene_name": "Uncharacterized protein",
  "term_id": "GO:0009306",
  "term_label": "protein secretion",
  "gene_symbol": "A0A2R8YE69",
  "gene": "UniProtKB:A0A2R8YE69"
}